regulation of pyrimidine-containing compound salvage [GO:1903930] (biological process) References: PMID:23695302 Sources: GOC:TermGenie, GO_REF:0000058 Also known as: regulation of pyrimidine salvage Definition: Any process that modulates the frequency, rate or extent of pyrimidine-containing compound salvage. Subtypes: GO:1903931 Relationships: is a type of regulation of biosynthetic process [GO:0009889]; regulates GO:0008655